{
  "gene_symbol": "LDB1",
  "term_id": "GO:0005634",
  "gene_name": "LIM domain-binding protein 1",
  "term_label": "nucleus",
  "gene": "UniProtKB:Q86U70"
}